{
  "gene": "UniProtKB:Q8IW35",
  "gene_name": "Centrosomal protein of 97 kDa",
  "term_label": "centrosome",
  "term_id": "GO:0005813",
  "gene_symbol": "CEP97"
}